{
  "term_label": "Unknown molecular function",
  "term_id": "UNKNOWN:0001",
  "gene": "UniProtKB:Q9NS93",
  "gene_symbol": "TM7SF3",
  "gene_name": "Transmembrane 7 superfamily member 3"
}